{
  "term_id": "GO:0005737",
  "gene_name": "tRNA-splicing endonuclease subunit Sen2",
  "gene_symbol": "TSEN2",
  "term_label": "cytoplasm",
  "gene": "UniProtKB:Q8NCE0"
}